{
  "gene": "UniProtKB:P0DMP2",
  "term_label": "regulation of synapse assembly",
  "gene_name": "SLIT-ROBO Rho GTPase-activating protein 2B",
  "term_id": "GO:0051963",
  "gene_symbol": "SRGAP2B"
}